{
  "gene": "UniProtKB:A0PK11",
  "term_id": "UNKNOWN:0003",
  "term_label": "Unknown cellular component",
  "gene_symbol": "CLRN2",
  "gene_name": "Clarin-2"
}